{
  "gene_name": "Immunoglobulin heavy variable 3_OR16-13 (non-functional) (Fragment)",
  "gene": "UniProtKB:A0A075B7E8",
  "gene_symbol": "IGHV3OR16-13",
  "term_label": "Unknown cellular component",
  "term_id": "UNKNOWN:0003"
}